{
  "gene": "UniProtKB:O15239",
  "gene_name": "NADH dehydrogenase [ubiquinone] 1 alpha subcomplex subunit 1",
  "gene_symbol": "NDUFA1",
  "term_label": "Unknown molecular function",
  "term_id": "UNKNOWN:0001"
}